positive regulation of homophilic cell adhesion [GO:1903387] (biological process) Also known as: up regulation of homophilic cell adhesion, up-regulation of homophilic cell adhesion, upregulation of homophilic cell adhesion, activation of homophilic cell adhesion Definition: Any process that activates or increases the frequency, rate or extent of homophilic cell adhesion. Relationships: is a type of positive regulation of cell-cell adhesion [GO:0022409]; is a type of regulation of homophilic cell adhesion [GO:1903385]; positively regulates homophilic cell-cell adhesion [GO:0007156] References: PMID:21724833 Sources: GOC:TermGenie, GOC:als, GO_REF:0000058